Rap protein signal transduction [GO:0032486] (biological process) Definition: An intracellular signaling cassette in which a small monomeric GTPase of the Rap subfamily relays a signal. Relationships: is_a small GTPase-mediated signal transduction [GO:0007264] Regulation: regulated by regulation of Rap protein signal transduction [GO:0032487] Sources: GOC:mah